{
  "term_id": "GO:0005634",
  "term_label": "nucleus",
  "gene": "UniProtKB:Q8N5A5",
  "gene_name": "Zinc finger CCCH-type with G patch domain-containing protein",
  "gene_symbol": "ZGPAT"
}